ribosomal S6-glutamic acid ligase activity [GO:0018169] (molecular function) Definition: Catalysis of the posttranslational transfer of one or more glutamic acid residues to the C-terminus of ribosomal protein S6. Relationships: is_a protein-glutamic acid ligase activity [GO:0070739] References: PMID:2570347 Sources: GOC:mah